{
  "term_id": "GO:0005615",
  "gene_name": "Neuroendocrine convertase 2",
  "gene": "UniProtKB:P16519",
  "term_label": "extracellular space",
  "gene_symbol": "PCSK2"
}